{
  "gene_symbol": "HPCAL4",
  "gene_name": "Hippocalcin-like protein 4",
  "gene": "UniProtKB:Q9UM19",
  "term_label": "Unknown cellular component",
  "term_id": "UNKNOWN:0003"
}